omega-amidase activity [GO:0050152] (molecular function) Relationships: is a type of hydrolase activity, acting on carbon-nitrogen (but not peptide) bonds, in linear amides [GO:0016811] Sources: EC:3.5.1.3, MetaCyc:OMEGA-AMIDASE-RXN Also known as: w-amidase activity, alpha-keto acid-omega-amidase activity, omega-amidodicarboxylate amidohydrolase activity Definition: Catalysis of the reaction: a monoamide of a dicarboxylic acid + H2O = a dicarboxylate + NH3.